response to dsDNA [GO:1990784] (biological process) Relationships: is a type of GO:1901698 References: PMID:10051633 Subtypes: cellular response to dsDNA [GO:1990786] Also known as: response to double-stranded DNA Definition: Any process that results in a change in state or activity of a cell or an organism (in terms of movement, secretion, enzyme production, gene expression, etc.) as a result of a double-stranded DNA stimulus.